{
  "gene_symbol": "PPIL6",
  "term_label": "Unknown molecular function",
  "gene": "UniProtKB:Q8IXY8",
  "term_id": "UNKNOWN:0001",
  "gene_name": "Probable inactive peptidyl-prolyl cis-trans isomerase-like 6"
}